{
  "gene_symbol": "CFAP298",
  "gene_name": "Cilia- and flagella-associated protein 298",
  "term_label": "Unknown biological process",
  "term_id": "UNKNOWN:0002",
  "gene": "UniProtKB:P57076"
}